{
  "gene": "UniProtKB:P42830",
  "term_id": "GO:0005615",
  "term_label": "extracellular space",
  "gene_symbol": "CXCL5",
  "gene_name": "C-X-C motif chemokine 5"
}